{
  "gene_name": "Olfactory receptor 5F1",
  "gene_symbol": "OR5F1",
  "gene": "UniProtKB:O95221",
  "term_id": "UNKNOWN:0002",
  "term_label": "Unknown biological process"
}